{
  "gene": "UniProtKB:Q9NVD7",
  "gene_symbol": "PARVA",
  "term_label": "cytoplasm",
  "gene_name": "Alpha-parvin",
  "term_id": "GO:0005737"
}